{
  "gene_symbol": "TGFBR3L",
  "term_label": "glycosaminoglycan binding",
  "term_id": "GO:0005539",
  "gene": "UniProtKB:H3BV60",
  "gene_name": "Transforming growth factor-beta receptor type 3-like protein"
}